{
  "gene_name": "COP9 signalosome complex subunit 3",
  "term_id": "GO:0006511",
  "gene_symbol": "COPS3",
  "gene": "UniProtKB:Q9UNS2",
  "term_label": "ubiquitin-dependent protein catabolic process"
}